{
  "gene": "UniProtKB:Q8NCY6",
  "gene_symbol": "MSANTD4",
  "term_label": "Unknown molecular function",
  "term_id": "UNKNOWN:0001",
  "gene_name": "Myb_SANT-like DNA-binding domain-containing protein 4"
}